{
  "gene_symbol": "FAM25A",
  "term_id": "UNKNOWN:0002",
  "gene": "UniProtKB:B3EWG3",
  "gene_name": "Protein FAM25A",
  "term_label": "Unknown biological process"
}